{
  "gene_symbol": "EPGN",
  "gene": "UniProtKB:Q6UW88",
  "term_label": "positive regulation of mitotic nuclear division",
  "gene_name": "Epigen",
  "term_id": "GO:0045840"
}